{
  "gene_symbol": "ITGAL",
  "term_label": "integrin alphaL-beta2 complex",
  "gene_name": "Integrin alpha-L",
  "term_id": "GO:0034687",
  "gene": "UniProtKB:P20701"
}